{
  "term_label": "angiogenesis",
  "gene_symbol": "PKNOX1",
  "gene_name": "Homeobox protein PKNOX1",
  "term_id": "GO:0001525",
  "gene": "UniProtKB:P55347"
}